{
  "term_label": "positive regulation of ERK1 and ERK2 cascade",
  "term_id": "GO:0070374",
  "gene_name": "Tyrosine-protein phosphatase non-receptor type 11",
  "gene_symbol": "PTPN11",
  "gene": "UniProtKB:Q06124"
}